{
  "gene": "UniProtKB:Q9C0G6",
  "gene_symbol": "DNAH6",
  "term_label": "dynein complex",
  "term_id": "GO:0030286",
  "gene_name": "Dynein axonemal heavy chain 6"
}